podosome [GO:0002102] (cellular component) Definition: An actin-rich adhesion structure characterized by formation upon cell substrate contact and localization at the substrate-attached part of the cell, contain an F-actin-rich core surrounded by a ring structure containing proteins such as vinculin and talin, and have a diameter of 0.5 mm. Note: Note that podosomes can be distinguished from other F-actin-rich structures or from other matrix contacts. For example, focal adhesions and focal contacts do not display a core structure of F-actin. Unlike focal adhesions, podosome assembly does not require de novo protein synthesis. However, most of the podosome ring components are found in focal adhesions and other cell-matrix contacts. Podosomes are typically found in cells that cross tissue boundaries, recruited to the leading edge of migrating cells, and are often sites of extracellular matrix degradation. References: PMID:12837608, PMID:15890982 Relationships: is a type of intracellular membraneless organelle [GO:0043232]; is part of actin cytoskeleton [GO:0015629]